{
  "gene_symbol": "RRP8",
  "gene": "UniProtKB:O43159",
  "term_label": "rDNA heterochromatin formation",
  "term_id": "GO:0000183",
  "gene_name": "Ribosomal RNA-processing protein 8"
}